D-nopaline dehydrogenase activity [GO:0047829] (molecular function) Definition: Catalysis of the reaction: D-nopaline + NADP+ + H2O = L-arginine + 2-oxoglutarate + NADPH + H+. Sources: RHEA:19637 Relationships: is a type of oxidoreductase activity, acting on the CH-NH group of donors, NAD or NADP as acceptor [GO:0016646] Also known as: 2-N-(D-1,3-dicarboxypropyl)-L-arginine:NADP+ oxidoreductase (L-arginine-forming), D-nopaline synthase activity, N2-(D-1,3-dicarboxypropyl)-L-arginine:NADP+ oxidoreductase (L-arginine-forming), NOS activity, nopaline dehydrogenase activity, nopaline synthase activity